{
  "gene": "UniProtKB:Q96LL3",
  "term_label": "Unknown molecular function",
  "gene_symbol": "FIMP",
  "gene_name": "Fertilization-influencing membrane protein",
  "term_id": "UNKNOWN:0001"
}